{
  "gene": "UniProtKB:Q5I0X4",
  "term_id": "UNKNOWN:0003",
  "term_label": "Unknown cellular component",
  "gene_symbol": "C6orf226",
  "gene_name": "Uncharacterized protein C6orf226"
}